{
  "gene_name": "Multifunctional procollagen lysine hydroxylase and glycosyltransferase LH3",
  "gene": "UniProtKB:O60568",
  "gene_symbol": "PLOD3",
  "term_label": "extracellular space",
  "term_id": "GO:0005615"
}